{
  "term_id": "UNKNOWN:0001",
  "gene_name": "Voltage-dependent calcium channel gamma-like subunit",
  "term_label": "Unknown molecular function",
  "gene": "UniProtKB:Q8WXS4",
  "gene_symbol": "TMEM37"
}